{
  "gene_name": "Sodium_bile acid cotransporter 5",
  "gene_symbol": "SLC10A5",
  "gene": "UniProtKB:Q5PT55",
  "term_label": "Unknown cellular component",
  "term_id": "UNKNOWN:0003"
}